response to muscle activity involved in regulation of muscle adaptation [GO:0014873] (biological process) Sources: GOC:ef, GOC:mtg_muscle Subtypes: GO:0014875 Also known as: response to fatigue, response to muscle activity involved in regulation of muscle plasticity Definition: Any process that results in a change in state or activity of a cell or an organism (in terms of movement, secretion, enzyme production, gene expression, etc.) as a result of a muscle activity stimulus. This process occurs as part of the regulation of muscle adaptation. Relationships: is a type of response to muscle activity [GO:0014850]; is a type of response to stimulus involved in regulation of muscle adaptation [GO:0014874]